{
  "term_label": "Unknown biological process",
  "term_id": "UNKNOWN:0002",
  "gene_name": "KICSTOR complex protein SZT2",
  "gene": "UniProtKB:Q5T011",
  "gene_symbol": "SZT2"
}